microglial cell mediated cytotoxicity [GO:0090634] (biological process) Relationships: is a type of leukocyte mediated cytotoxicity [GO:0001909]; is_a myeloid leukocyte mediated immunity [GO:0002444] References: PMID:19100238 Sources: GOC:BHF, GOC:nc Definition: The directed killing of a target cell by a microglial cell. Regulation: regulated by regulation of microglial cell mediated cytotoxicity [GO:1904149]; negatively regulated by GO:1904150; positively regulated by GO:1904151